sepal morphogenesis [GO:0048447] (biological process) Definition: The process in which the anatomical structures of the sepal are generated and organized. Relationships: is a type of floral organ morphogenesis [GO:0048444]; is part of sepal development [GO:0048442] Sources: GOC:go_curators